narrow pore channel activity [GO:0022842] (molecular function) Relationships: is a type of channel activity [GO:0015267] Sources: GOC:mtg_transport, ISBN:0815340729 Subtypes: narrow pore, gated channel activity [GO:0022831], leak channel activity [GO:0022840] Definition: Enables the transport of a solute across a membrane via a narrow pore channel that may be gated or ungated.